{
  "term_id": "GO:0003712",
  "term_label": "transcription coregulator activity",
  "gene_name": "RNA-binding protein EWS",
  "gene": "UniProtKB:Q01844",
  "gene_symbol": "EWSR1"
}